meiotic G2/MI DNA replication checkpoint signaling [GO:0033315] (biological process) Relationships: is a type of GO:0000076; is a type of meiotic DNA integrity checkpoint signaling [GO:0044778]; is a type of negative regulation of G2/MI transition of meiotic cell cycle [GO:0110031]; happens during GO:0051331 Sources: GOC:mtg_cell_cycle Definition: A signal transduction process that controls the G2/M1 transition of the meiotic cell cycle and prevents the initiation of nuclear division until DNA replication is complete. Also known as: meiotic G2/MI DNA replication checkpoint, meiotic cell cycle DNA replication checkpoint, signal transduction involved in meiotic DNA replication checkpoint